{
  "gene_name": "Syntaxin-3",
  "gene_symbol": "STX3",
  "term_id": "GO:0098794",
  "term_label": "postsynapse",
  "gene": "UniProtKB:Q13277"
}